{
  "term_label": "neuropeptide signaling pathway",
  "gene": "UniProtKB:Q9HCQ7",
  "gene_symbol": "NPVF",
  "gene_name": "Pro-FMRFamide-related neuropeptide VF",
  "term_id": "GO:0007218"
}